{
  "gene": "UniProtKB:Q01118",
  "gene_symbol": "SCN7A",
  "term_id": "GO:0035725",
  "term_label": "sodium ion transmembrane transport",
  "gene_name": "Sodium channel protein type 7 subunit alpha"
}